{
  "gene_symbol": "USP17L12",
  "gene": "UniProtKB:C9JPN9",
  "gene_name": "Ubiquitin carboxyl-terminal hydrolase 17-like protein 12",
  "term_id": "GO:0031647",
  "term_label": "regulation of protein stability"
}